{
  "gene_name": "Ras-specific guanine nucleotide-releasing factor RalGPS2",
  "gene_symbol": "RALGPS2",
  "term_id": "GO:0032485",
  "gene": "UniProtKB:Q86X27",
  "term_label": "regulation of Ral protein signal transduction"
}